negative regulation of abscisic acid biosynthetic process [GO:0090359] (biological process) Also known as: negative regulation of abscisic acid biosynthesis Definition: Any process that decreases the frequency, rate or extent of the chemical reactions and pathways resulting in the formation of abscisic acid. Sources: GOC:tb Relationships: is a type of regulation of abscisic acid biosynthetic process [GO:0010115]; is a type of negative regulation of isoprenoid metabolic process [GO:0045827]; is a type of negative regulation of lipid biosynthetic process [GO:0051055]; is a type of negative regulation of alcohol biosynthetic process [GO:1902931]; negatively regulates GO:0009688